meiotic septin complex [GO:0032152] (CC) References: PMID:16009555 Sources: GOC:krc Definition: A heterooligomeric septin complex that acts during meiotic cell division. Relationships: is a type of septin complex [GO:0031105]